{
  "gene_name": "JmjC domain-containing protein 8",
  "gene": "UniProtKB:Q96S16",
  "term_id": "GO:0005634",
  "gene_symbol": "JMJD8",
  "term_label": "nucleus"
}